{
  "gene": "UniProtKB:Q9H4A6",
  "term_id": "GO:0043001",
  "gene_name": "Golgi phosphoprotein 3",
  "gene_symbol": "GOLPH3",
  "term_label": "Golgi to plasma membrane protein transport"
}